regulation of protein localization to cell periphery [GO:1904375] (biological process) Definition: Any process that modulates the frequency, rate or extent of protein localization to cell periphery. Relationships: is a type of regulation of protein localization [GO:0032880]; regulates protein localization to cell periphery [GO:1990778] References: PMID:18216290 Sources: GOC:TermGenie, GO_REF:0000058 Subtypes: regulation of neurotransmitter receptor localization to postsynaptic specialization membrane [GO:0098696], regulation of exocytic insertion of neurotransmitter receptor to postsynaptic membrane [GO:0099145], regulation of protein localization to plasma membrane [GO:1903076], GO:1903567, negative regulation of protein localization to cell periphery [GO:1904376], positive regulation of protein localization to cell periphery [GO:1904377], regulation of protein localization to basolateral plasma membrane [GO:1904508], regulation of protein localization to cell cortex [GO:1904776]